{
  "gene": "UniProtKB:Q9BWJ5",
  "gene_symbol": "SF3B5",
  "term_label": "precatalytic spliceosome",
  "term_id": "GO:0071011",
  "gene_name": "Splicing factor 3B subunit 5"
}